{
  "gene_name": "Cdc42-interacting protein 4",
  "term_id": "UNKNOWN:0003",
  "term_label": "Unknown cellular component",
  "gene_symbol": "TRIP10",
  "gene": "UniProtKB:Q15642"
}